{
  "term_id": "UNKNOWN:0002",
  "gene_name": "Glutamate-rich protein 6B",
  "gene": "UniProtKB:Q5W0A0",
  "term_label": "Unknown biological process",
  "gene_symbol": "ERICH6B"
}